{
  "gene_name": "Protein PHTF1",
  "term_id": "UNKNOWN:0003",
  "term_label": "Unknown cellular component",
  "gene_symbol": "PHTF1",
  "gene": "UniProtKB:Q9UMS5"
}